cellular response to gastrin [GO:1990878] (biological process) Definition: Any process that results in a change in state or activity of a cell (in terms of movement, secretion, enzyme production, gene expression, etc.) as a result of a gastrin stimulus. References: PMID:10348814 Relationships: is a type of cellular response to peptide hormone stimulus [GO:0071375]; is a type of response to gastrin [GO:1990867]